{
  "gene_symbol": "SMPD2",
  "gene_name": "Sphingomyelin phosphodiesterase 2",
  "gene": "UniProtKB:O60906",
  "term_id": "GO:0004767",
  "term_label": "sphingomyelin phosphodiesterase activity"
}